sterol metabolic process [GO:0016125] (BP) Sources: ISBN:0198547684 Relationships: is a type of steroid metabolic process [GO:0008202] Definition: The chemical reactions and pathways involving sterols, steroids with one or more hydroxyl groups and a hydrocarbon side-chain in the molecule. Subtypes: cholesterol metabolic process [GO:0008203], ergosterol metabolic process [GO:0008204], GO:0008205, GO:0016126, sterol catabolic process [GO:0016127], GO:0036196 Also known as: sterol metabolism